{
  "gene_symbol": "PON1",
  "term_id": "GO:0009636",
  "term_label": "response to toxic substance",
  "gene_name": "Serum paraoxonase_arylesterase 1",
  "gene": "UniProtKB:P27169"
}